maltose biosynthetic process [GO:0000024] (biological process) Definition: The chemical reactions and pathways resulting in the formation of the disaccharide maltose (4-O-alpha-D-glucopyranosyl-D-glucopyranose). Sources: GOC:jl, ISBN:0198506732 Relationships: is_a GO:0000023; is_a disaccharide biosynthetic process [GO:0046351] Also known as: malt sugar biosynthesis, malt sugar biosynthetic process, maltose anabolism, maltose biosynthesis, maltose formation, maltose synthesis